{
  "term_id": "UNKNOWN:0003",
  "gene_symbol": "LZTS2",
  "gene": "UniProtKB:Q9BRK4",
  "term_label": "Unknown cellular component",
  "gene_name": "Leucine zipper putative tumor suppressor 2"
}